{
  "gene": "UniProtKB:Q96GD4",
  "term_label": "midbody",
  "gene_symbol": "AURKB",
  "gene_name": "Aurora kinase B",
  "term_id": "GO:0030496"
}